{
  "term_label": "plasma membrane",
  "gene_symbol": "ATP11B",
  "gene": "UniProtKB:Q9Y2G3",
  "gene_name": "Phospholipid-transporting ATPase IF",
  "term_id": "GO:0005886"
}